{
  "term_id": "GO:0061564",
  "gene_symbol": "OLIG2",
  "term_label": "axon development",
  "gene": "UniProtKB:Q13516",
  "gene_name": "Oligodendrocyte transcription factor 2"
}